amine sulfotransferase activity [GO:0047685] (molecular function) Also known as: amine sulphotransferase activity, arylamine sulfotransferase activity, 3'-phosphoadenylyl-sulfate:amine N-sulfotransferase activity, amine N-sulfotransferase activity Definition: Catalysis of the reaction: 3'-phosphoadenosine 5'-phosphosulfate + an amine = adenosine 3',5'-bisphosphate + a sulfamate. Sources: EC:2.8.2.3, MetaCyc:ARYLAMINE-SULFOTRANSFERASE-RXN Relationships: is a type of sulfotransferase activity [GO:0008146]